{
  "term_label": "Unknown biological process",
  "gene_symbol": "PPP2R3B",
  "gene_name": "Serine_threonine-protein phosphatase 2A regulatory subunit B'' subunit beta",
  "term_id": "UNKNOWN:0002",
  "gene": "UniProtKB:Q9Y5P8"
}